{
  "gene_symbol": "TTK",
  "term_label": "mitotic spindle assembly checkpoint signaling",
  "gene_name": "Dual specificity protein kinase TTK",
  "term_id": "GO:0007094",
  "gene": "UniProtKB:P33981"
}